regulation of metanephric DCT cell differentiation [GO:2000592] (biological process) Subtypes: negative regulation of metanephric DCT cell differentiation [GO:2000593], positive regulation of metanephric DCT cell differentiation [GO:2000594] Definition: Any process that modulates the frequency, rate or extent of metanephric DCT cell differentiation. Sources: GOC:obol Also known as: regulation of metanephric distal convoluted tubule cell differentiation Relationships: is a type of regulation of cell differentiation [GO:0045595]; regulates metanephric DCT cell differentiation [GO:0072240]